prostate glandular acinus morphogenesis [GO:0060526] (biological process) Sources: GOC:dph Definition: The process in which the prostate glandular acini are generated and organized. The glandular acini are the saclike structures of the gland. Relationships: is a type of GO:0060740; is part of GO:0060525